{
  "gene": "UniProtKB:P06400",
  "gene_name": "Retinoblastoma-associated protein",
  "term_label": "negative regulation of G1/S transition of mitotic cell cycle",
  "gene_symbol": "RB1",
  "term_id": "GO:2000134"
}